{
  "gene_name": "Histone-binding protein RBBP7",
  "gene": "UniProtKB:Q16576",
  "gene_symbol": "RBBP7",
  "term_id": "GO:0005634",
  "term_label": "nucleus"
}